L-arabinose isomerase activity [GO:0008733] (molecular function) Also known as: L-arabinose aldose-ketose-isomerase activity, L-arabinose ketol-isomerase activity Sources: EC:5.3.1.4, RHEA:14821 Relationships: is a type of intramolecular oxidoreductase activity, interconverting aldoses and ketoses [GO:0016861] Definition: Catalysis of the reaction: L-arabinose = L-ribulose.